pallium development [GO:0021543] (biological process) References: PMID:12626695 Sources: GOC:cls, GOC:dgh, GOC:dph, GOC:jid, GO_REF:0000021 Relationships: is a type of anatomical structure development [GO:0048856]; is part of GO:0021537 Definition: The process whose specific outcome is the progression of the pallium over time, from its formation to the mature structure. The pallium is the roof region of the telencephalon.